proteasome activator complex [GO:0008537] (cellular component) Definition: A multisubunit complex that activates the hydrolysis of small nonubiquitinated peptides by binding to the proteasome core complex. Relationships: is_a protein-containing complex [GO:0032991]; is part of proteasome accessory complex [GO:0022624] Also known as: PA28 Sources: GOC:rb